interleukin-11 production [GO:0032614] (BP) Relationships: is a type of cytokine production [GO:0001816] Definition: The appearance of interleukin-11 due to biosynthesis or secretion following a cellular stimulus, resulting in an increase in its intracellular or extracellular levels. Regulation: regulated by regulation of interleukin-11 production [GO:0032654]; negatively regulated by negative regulation of interleukin-11 production [GO:0032694]; positively regulated by GO:0032734 Sources: GOC:mah Also known as: IL-11 production, interleukin-11 biosynthetic process, interleukin-11 secretion